regulation of positive chemotaxis to cAMP by DIF-2 [GO:0061121] (biological process) Definition: Any process that modulates the rate, frequency, or extent of directed movement of a motile cell or organism up a concentration gradient of 3',5'-cAMP by the action of DIF-2. DIF-2 is a chlorinated alkylphenone. Relationships: is a type of regulation of positive chemotaxis to cAMP by chlorinated alkylphenone [GO:0061119] Subtypes: positive regulation of chemotaxis to cAMP by DIF-2 [GO:0061128], negative regulation of positive chemotaxis to cAMP by DIF-2 [GO:0061129] Sources: GOC:dph